{
  "term_label": "catalytic step 2 spliceosome",
  "gene_symbol": "SNRPG",
  "gene_name": "Small nuclear ribonucleoprotein G",
  "term_id": "GO:0071013",
  "gene": "UniProtKB:P62308"
}